mitochondrial RNA 5'-end processing [GO:0000964] (biological process) Also known as: mitochondrial RNA 5' end processing Relationships: is a type of mitochondrial RNA processing [GO:0000963]; is a type of GO:0000966 Subtypes: mitochondrial tRNA 5'-end processing [GO:0097745] Definition: Any process involved in forming the mature 5' end of an RNA molecule transcribed from a mitochondrial genome; occurs in the mitochondrion. Sources: GOC:krc, GOC:mah